{
  "term_label": "Unknown biological process",
  "gene_name": "Testis-specific Y-encoded protein 4",
  "gene": "UniProtKB:P0CV99",
  "gene_symbol": "TSPY4",
  "term_id": "UNKNOWN:0002"
}